prostaglandin E2 9-reductase activity [GO:0050221] (molecular function) Sources: EC:1.1.1.189, MetaCyc:PROSTAGLANDIN-E2-9-REDUCTASE-RXN Also known as: (5Z,13E)-(15S)-9alpha,11alpha,15-trihydroxyprosta-5,13-dienoate:NADP+ 9-oxidoreductase activity, 9-keto-prostaglandin E(2) reductase activity, 9-keto-prostaglandin E2 reductase activity, 9-ketoprostaglandin reductase activity, PGE(2) 9-ketoreductase activity, PGE(2) 9-oxoreductase activity, PGE-9-ketoreductase activity, PGE2 9-ketoreductase activity, PGE2 9-oxoreductase activity, PGE2-9-OR, PGE2-9-ketoreductase activity, prostaglandin E 9-ketoreductase activity, prostaglandin E2-9-oxoreductase activity, prostaglandin-E(2) 9-oxoreductase activity, prostaglandin-E2 9-oxoreductase activity, reductase, 15-hydroxy-9-oxoprostaglandin Definition: Catalysis of the reaction: (5Z,13E)-(15S)-9-alpha,11-alpha,15-trihydroxyprosta-5,13-dienoate + NADP+ = (5Z,13E)-(15S)-11-alpha,15-dihydroxy-9-oxoprosta-5,13-dienoate + NADPH. Relationships: is a type of oxidoreductase activity, acting on the CH-OH group of donors, NAD or NADP as acceptor [GO:0016616]